{
  "gene_symbol": "UPRT",
  "term_id": "UNKNOWN:0002",
  "gene": "UniProtKB:Q96BW1",
  "gene_name": "Uracil phosphoribosyltransferase homolog",
  "term_label": "Unknown biological process"
}